COPI-coated Golgi to ER transport vesicle [GO:0030142] (cellular component) Also known as: Golgi to ER constitutive secretory pathway transport vesicle, Golgi to endoplasmic reticulum transport vesicle, Golgi-ER transport vesicle, Golgi-endoplasmic reticulum transport vesicle, retrograde transport vesicle Definition: A vesicle that mediates transport from the Golgi to the endoplasmic reticulum. Relationships: is a type of GO:0030133; is a type of GO:0030137 References: PMID:22160157 Sources: GOC:mah